{
  "gene_name": "Endoplasmic reticulum-Golgi intermediate compartment protein 3",
  "term_label": "Golgi membrane",
  "gene": "UniProtKB:Q9Y282",
  "gene_symbol": "ERGIC3",
  "term_id": "GO:0000139"
}